{
  "term_id": "UNKNOWN:0001",
  "gene_name": "Immunoglobulin kappa variable 1D-12",
  "term_label": "Unknown molecular function",
  "gene_symbol": "IGKV1D-12",
  "gene": "UniProtKB:P01611"
}